{
  "term_id": "UNKNOWN:0003",
  "gene_symbol": "C10orf105",
  "gene_name": "Uncharacterized protein C10orf105",
  "term_label": "Unknown cellular component",
  "gene": "UniProtKB:Q8TEF2"
}